{
  "gene": "UniProtKB:A0A6Q8PHA8",
  "term_label": "Unknown molecular function",
  "gene_name": "Uncharacterized protein",
  "term_id": "UNKNOWN:0001",
  "gene_symbol": "A0A6Q8PHA8"
}